{
  "gene_name": "Retinoic acid-induced protein 2",
  "term_label": "Unknown molecular function",
  "gene_symbol": "RAI2",
  "gene": "UniProtKB:Q9Y5P3",
  "term_id": "UNKNOWN:0001"
}